{
  "gene_symbol": "WDR45",
  "gene_name": "WD repeat domain phosphoinositide-interacting protein 4",
  "term_id": "GO:0000425",
  "term_label": "pexophagy",
  "gene": "UniProtKB:Q9Y484"
}